{
  "gene": "UniProtKB:O75388",
  "gene_symbol": "GPR32",
  "term_id": "GO:0007200",
  "term_label": "phospholipase C-activating G protein-coupled receptor signaling pathway",
  "gene_name": "Probable G-protein coupled receptor 32"
}